{
  "gene_symbol": "E2F4",
  "term_label": "DNA-binding transcription factor activity, RNA polymerase II-specific",
  "gene": "UniProtKB:Q16254",
  "term_id": "GO:0000981",
  "gene_name": "Transcription factor E2F4"
}